peg and socket contact [GO:0044286] (cellular component) Relationships: is a type of cell-cell contact zone [GO:0044291] References: PMID:12883993, PMID:16166562, PMID:17591898 Sources: GOC:tfm, NIF_Subcellular:sao1943947957 Definition: A cell-cell contact zone that consists of membrane invaginations extending from either cell, which contain tight-, gap-, and adherens junctions. Peg and socket contacts form between endothelial cells and pericytes, and between lens fiber cells. Also known as: ball and socket contact